{
  "gene_name": "SET domain-containing protein 9",
  "term_label": "Unknown biological process",
  "gene_symbol": "SETD9",
  "term_id": "UNKNOWN:0002",
  "gene": "UniProtKB:Q8NE22"
}